{
  "gene_name": "T-complex protein 1 subunit zeta",
  "term_id": "GO:0006457",
  "gene": "UniProtKB:P40227",
  "gene_symbol": "CCT6A",
  "term_label": "protein folding"
}